{
  "gene": "UniProtKB:Q8N2R8",
  "term_label": "Unknown cellular component",
  "term_id": "UNKNOWN:0003",
  "gene_name": "Protein FAM43A",
  "gene_symbol": "FAM43A"
}